{
  "gene_name": "Brain acid soluble protein 1",
  "term_label": "transcription corepressor activity",
  "gene": "UniProtKB:P80723",
  "term_id": "GO:0003714",
  "gene_symbol": "BASP1"
}